{
  "term_id": "GO:0043325",
  "gene_symbol": "DAPP1",
  "term_label": "phosphatidylinositol-3,4-bisphosphate binding",
  "gene_name": "Dual adapter for phosphotyrosine and 3-phosphotyrosine and 3-phosphoinositide",
  "gene": "UniProtKB:Q9UN19"
}